{
  "term_label": "GTPase activity",
  "gene_symbol": "GBP3",
  "gene": "UniProtKB:Q9H0R5",
  "gene_name": "Guanylate-binding protein 3",
  "term_id": "GO:0003924"
}